chloroplast organization [GO:0009658] (biological process) Subtypes: chloroplast relocation [GO:0009902], chloroplast fission [GO:0010020], chloroplast elongation [GO:0010151], GO:1904821 Sources: GOC:jid Relationships: is_a GO:0009657 Definition: A process that is carried out at the cellular level which results in the assembly, arrangement of constituent parts, or disassembly of the chloroplast. Also known as: chloroplast organisation, chloroplast organization and biogenesis